{
  "gene_symbol": "PALLD",
  "gene": "UniProtKB:Q8WX93",
  "term_label": "dendrite self-avoidance",
  "gene_name": "Palladin",
  "term_id": "GO:0070593"
}